positive regulation of icosanoid secretion [GO:0032305] (biological process) Sources: GOC:mah Relationships: is a type of regulation of icosanoid secretion [GO:0032303]; is a type of positive regulation of secretion [GO:0051047]; is a type of GO:2000193; positively regulates GO:0032309 Also known as: positive regulation of eicosanoid secretion, up regulation of icosanoid secretion, up-regulation of icosanoid secretion, upregulation of icosanoid secretion, activation of icosanoid secretion, stimulation of icosanoid secretion Definition: Any process that activates or increases the frequency, rate or extent of the controlled release of an icosanoid from a cell. Subtypes: GO:0032308, GO:0090238